{
  "term_label": "Unknown cellular component",
  "term_id": "UNKNOWN:0003",
  "gene_symbol": "C14orf132",
  "gene": "UniProtKB:Q9NPU4",
  "gene_name": "Uncharacterized protein C14orf132"
}